isocitrate-homoisocitrate dehydrogenase activity [GO:0033708] (molecular function) Relationships: is a type of oxidoreductase activity, acting on the CH-OH group of donors, NAD or NADP as acceptor [GO:0016616] Also known as: PH1722, homoisocitrate-isocitrate dehydrogenase activity, isocitrate(homoisocitrate):NAD+ oxidoreductase (decarboxylating) activity Definition: Catalysis of the reactions: isocitrate + NAD+ = 2-oxoglutarate + CO2 + NADH, and (1R,2S)-1-hydroxybutane-1,2,4-tricarboxylate + NAD+ = 2-oxoadipate + CO2 + NADH + H+. Sources: EC:1.1.1.286